positive regulation of iron ion transport [GO:0034758] (biological process) Definition: Any process that activates or increases the frequency, rate or extent of the directed movement of iron ions into, out of or within a cell, or between cells, by means of some agent such as a transporter or pore. Sources: GOC:mah Also known as: positive regulation of iron transport, up regulation of iron ion transport, up-regulation of iron ion transport, upregulation of iron ion transport, activation of iron ion transport, stimulation of iron ion transport Relationships: is_a GO:0034756; is a type of positive regulation of monoatomic ion transport [GO:0043270]; positively regulates iron ion transport [GO:0006826] Subtypes: GO:0034761